protein adenylylhydrolase activity [GO:0044603] (MF) References: PMID:21734656 Relationships: is a type of GO:0008081; is a type of catalytic activity, acting on a protein [GO:0140096] Also known as: protein deAMPylase activity, protein deAMPylation activity Definition: Catalysis of the reaction: adenylyl-protein+ H2O = adenylate + protein; mediates the removal of an adenylyl (adenosine 5'-monophosphate; AMP group) from specific residues of target proteins.